glucagon receptor activity [GO:0004967] (molecular function) References: PMID:22438981 Sources: GOC:mah, GOC:signaling Definition: Combining with glucagon and transmitting the signal across the membrane by activating an associated G-protein; promotes the exchange of GDP for GTP on the alpha subunit of a heterotrimeric G-protein complex. Relationships: is a type of G protein-coupled peptide receptor activity [GO:0008528]; is part of GO:0071377